neural crest cell fate specification [GO:0014036] (biological process) Relationships: is a type of stem cell fate specification [GO:0048866]; is part of neural crest cell fate commitment [GO:0014034] Definition: The process in which a cell becomes capable of differentiating autonomously into a neural crest cell in an environment that is neutral with respect to the developmental pathway; upon specification, the cell fate can be reversed. Regulation: RO_0002211 by GO:1905295; negatively regulated by negative regulation of neural crest cell fate specification [GO:1905296]; positively regulated by positive regulation of neural crest cell fate specification [GO:1905297] Sources: GOC:dh, GOC:ef